{
  "term_label": "myelination",
  "gene_name": "Myelin and lymphocyte protein",
  "gene": "UniProtKB:P21145",
  "term_id": "GO:0042552",
  "gene_symbol": "MAL"
}